{
  "gene": "UniProtKB:P19876",
  "term_label": "Unknown biological process",
  "gene_name": "C-X-C motif chemokine 3",
  "gene_symbol": "CXCL3",
  "term_id": "UNKNOWN:0002"
}